{
  "gene_symbol": "ANLN",
  "gene_name": "Anillin",
  "term_id": "GO:0005826",
  "gene": "UniProtKB:Q9NQW6",
  "term_label": "actomyosin contractile ring"
}